{
  "gene": "UniProtKB:Q96E66",
  "term_label": "axoneme",
  "gene_name": "Leucine-rich repeat-containing protein 51",
  "gene_symbol": "LRRC51",
  "term_id": "GO:0005930"
}